{
  "gene_name": "Methyltransferase-like 26",
  "term_id": "UNKNOWN:0001",
  "term_label": "Unknown molecular function",
  "gene_symbol": "METTL26",
  "gene": "UniProtKB:Q96S19"
}